{
  "gene": "UniProtKB:Q6PII3",
  "gene_name": "Coiled-coil domain-containing protein 174",
  "term_id": "GO:0005634",
  "gene_symbol": "CCDC174",
  "term_label": "nucleus"
}